{
  "term_id": "GO:0019955",
  "gene": "UniProtKB:Q99062",
  "term_label": "cytokine binding",
  "gene_name": "Granulocyte colony-stimulating factor receptor",
  "gene_symbol": "CSF3R"
}